{
  "gene_symbol": "PDZD2",
  "gene": "UniProtKB:O15018",
  "gene_name": "PDZ domain-containing protein 2",
  "term_id": "UNKNOWN:0001",
  "term_label": "Unknown molecular function"
}